chemokine (C-X-C motif) ligand 16 production [GO:0097392] (biological process) Definition: The appearance of chemokine (C-X-C motif) ligand 16 (CXCL16) due to biosynthesis or secretion following a cellular stimulus, resulting in an increase in its intracellular or extracellular levels. Sources: GOC:rv Relationships: is a type of chemokine production [GO:0032602] Also known as: CXCL16 production